{
  "term_label": "histone deacetylase binding",
  "term_id": "GO:0042826",
  "gene_symbol": "MAGEA11",
  "gene_name": "Melanoma-associated antigen 11",
  "gene": "UniProtKB:P43364"
}